{
  "gene": "UniProtKB:Q6DD88",
  "gene_name": "Atlastin-3",
  "term_label": "GTP binding",
  "term_id": "GO:0005525",
  "gene_symbol": "ATL3"
}